cysteine export across plasma membrane [GO:0033228] (biological process) Relationships: is a type of amino acid export across plasma membrane [GO:0032973]; is a type of cysteine transmembrane transport [GO:1903712] Sources: GOC:mlg Also known as: cysteine export Definition: The directed movement of cysteine from inside of a cell, across the plasma membrane and into the extracellular region.